{
  "gene": "UniProtKB:Q92959",
  "term_id": "GO:0043252",
  "gene_name": "Solute carrier organic anion transporter family member 2A1",
  "term_label": "sodium-independent organic anion transport",
  "gene_symbol": "SLCO2A1"
}